negative regulation of mitotic cell cycle, embryonic [GO:0045976] (biological process) Definition: Any process that stops, prevents or reduces the rate or extent of progression through the embryonic mitotic cell cycle. Also known as: down regulation of progression through embryonic mitotic cell cycle, down-regulation of progression through embryonic mitotic cell cycle, downregulation of progression through embryonic mitotic cell cycle, negative regulation of embryonic mitotic cell cycle, negative regulation of embryonic mitotic cell cycle progression, negative regulation of progression through embryonic mitotic cell cycle, inhibition of progression through embryonic mitotic cell cycle Sources: GOC:dph, GOC:go_curators, GOC:tb Relationships: is a type of regulation of mitotic cell cycle, embryonic [GO:0009794]; is a type of negative regulation of mitotic cell cycle [GO:0045930]; negatively regulates GO:0045448 Subtypes: GO:0046001, negative regulation of syncytial blastoderm mitotic cell cycle [GO:0046003]